denatured protein binding [GO:0031249] (molecular function) Relationships: is_a protein binding [GO:0005515] Note: Note that this term should not be confused with 'unfolded protein binding ; GO:0051082', which usually refers to proteins that have not yet folded into their active states. Denatured proteins once were in their correct functional conformations, but have become incorrectly folded, and often form aggregates. Sources: GOC:mlg Definition: Binding to a denatured protein.